{
  "gene_name": "Interleukin-37",
  "term_id": "GO:0005615",
  "gene": "UniProtKB:Q9NZH6",
  "gene_symbol": "IL37",
  "term_label": "extracellular space"
}